{
  "term_id": "GO:0005737",
  "term_label": "cytoplasm",
  "gene_symbol": "EHD4",
  "gene": "UniProtKB:Q9H223",
  "gene_name": "EH domain-containing protein 4"
}